N-acetylneuraminylgalactosylglucosylceramide beta-1,4-N-acetylgalactosaminyltransferase activity [GO:0047233] (molecular function) Sources: RHEA:81947 Relationships: is a type of GO:0008376 Also known as: UDP-N-acetyl-D-galactosamine:N-acetylneuraminyl-2,3-alpha-D-galactosyl-1,4-beta-D-glucosylceramide beta-1,4-N-acetylgalactosaminyltransferase activity, uridine diphosphoacetylgalactosamine-acetylneuraminyl(alpha2->3)galactosyl(beta1->4)glucosyl beta1->4-acetylgalactosaminyltransferase activity Definition: Catalysis of the reaction: an N-acetyl-alpha-neuraminyl-(2->3)-beta-D-galactosyl derivative + UDP-N-acetyl-alpha-D-galactosamine = an N-acetyl-beta-D-galactosaminyl-(1->4)-[N-acetyl-alpha-neuraminyl-(2->3)]-beta-D-galactosyl derivative + UDP + H+.